L-histidine N-acetyltransferase activity [GO:0047981] (molecular function) Relationships: is_a GO:0140085 Also known as: histidine N-acetyltransferase activity, acetyl-CoA:L-histidine N-acetyltransferase activity, acetylhistidine synthetase activity, histidine acetyltransferase activity Sources: EC:2.3.1.33, RHEA:24596 Definition: Catalysis of the reaction: L-histidine + acetyl-CoA = N(alpha)-acetyl-L-histidine + CoA + H+.